{
  "gene": "UniProtKB:P27987",
  "gene_name": "Inositol-trisphosphate 3-kinase B",
  "term_id": "GO:0046854",
  "term_label": "phosphatidylinositol phosphate biosynthetic process",
  "gene_symbol": "ITPKB"
}